embryonic digit morphogenesis [GO:0042733] (biological process) Sources: GOC:bf, GOC:jl, UBERON:0002544 Relationships: is a type of embryonic morphogenesis [GO:0048598]; is part of embryonic limb morphogenesis [GO:0030326] Definition: The process, occurring in the embryo, by which the anatomical structures of the digit are generated and organized. A digit is one of the terminal divisions of an appendage, such as a finger or toe.